{
  "term_label": "cytosol",
  "term_id": "GO:0005829",
  "gene_symbol": "METTL21A",
  "gene": "UniProtKB:Q8WXB1",
  "gene_name": "Protein N-lysine methyltransferase METTL21A"
}